{
  "gene_name": "T cell receptor beta variable 30",
  "gene_symbol": "TRBV30",
  "term_label": "Unknown molecular function",
  "gene": "UniProtKB:A0A0K0K1B3",
  "term_id": "UNKNOWN:0001"
}